negative regulation of cardioblast cell fate specification [GO:0009997] (biological process) Sources: GOC:go_curators Relationships: is a type of regulation of cardioblast cell fate specification [GO:0042686]; is a type of negative regulation of cardioblast differentiation [GO:0051892]; is a type of negative regulation of cardiac cell fate specification [GO:2000044]; negatively regulates cardioblast cell fate specification [GO:0042685] Definition: Any process that restricts, stops or prevents a cell from specifying into a cardioblast. A cardioblast is a cardiac precursor cell. It is a cell that has been committed to a cardiac fate, but will undergo more cell division rather than terminally differentiating. Also known as: down regulation of cardioblast cell fate specification, down-regulation of cardioblast cell fate specification, downregulation of cardioblast cell fate specification, suppression of cardioblast cell fate, inhibition of cardioblast cell fate specification